terpenoid transport [GO:0046865] (biological process) Definition: The directed movement of terpenoids into, out of or within a cell, or between cells, by means of some agent such as a transporter or pore. Terpenoids are a class of compounds characterized by an isoprenoid chemical structure and include derivatives with various functional groups. Sources: GOC:ai Relationships: is a type of isoprenoid transport [GO:0046864] Subtypes: GO:0034633, juvenile hormone secretion [GO:0045443], GO:0046866, GO:0071938, abscisic acid transport [GO:0080168], gibberellic acid transmembrane transport [GO:1905200]